{
  "gene_symbol": "MATN3",
  "term_id": "UNKNOWN:0001",
  "gene": "UniProtKB:O15232",
  "gene_name": "Matrilin-3",
  "term_label": "Unknown molecular function"
}